{
  "term_id": "GO:0030550",
  "term_label": "acetylcholine receptor inhibitor activity",
  "gene_name": "Lymphocyte antigen 6H",
  "gene_symbol": "LY6H",
  "gene": "UniProtKB:O94772"
}